{
  "gene_name": "Negative elongation factor E",
  "term_label": "negative regulation of transcription elongation by RNA polymerase II",
  "gene_symbol": "NELFE",
  "term_id": "GO:0034244",
  "gene": "UniProtKB:P18615"
}